{
  "term_label": "Unknown biological process",
  "gene_name": "Storkhead-box protein 2",
  "gene": "UniProtKB:Q9P2F5",
  "gene_symbol": "STOX2",
  "term_id": "UNKNOWN:0002"
}